cytoskeleton polarization involved in growth plate cartilage chondrocyte division [GO:0003426] (biological process) Relationships: is a type of establishment or maintenance of cytoskeleton polarity [GO:0030952]; is part of establishment of cell polarity involved in growth plate cartilage chondrocyte division [GO:0003424] Sources: GOC:ascb_2009, GOC:dph, GOC:tb Definition: A process that is carried out at the cellular level which results in the polarization of cytoskeletal structures in a growth plate cartilage chondrocyte. This process results in the oriented division of the cell. Regulation: regulated by regulation of cytoskeleton polarization involved in growth plate cartilage chondrocyte division [GO:0003427] Subtypes: establishment of mitotic spindle orientation involved in growth plate cartilage chondrocyte division [GO:0003425]